{
  "gene_name": "Potassium voltage-gated channel subfamily H member 5",
  "gene_symbol": "KCNH5",
  "term_id": "GO:0005249",
  "term_label": "voltage-gated potassium channel activity",
  "gene": "UniProtKB:Q8NCM2"
}